{
  "gene_symbol": "RREB1",
  "term_id": "GO:0006357",
  "term_label": "regulation of transcription by RNA polymerase II",
  "gene_name": "Ras-responsive element-binding protein 1",
  "gene": "UniProtKB:Q92766"
}